{
  "gene_symbol": "SNX11",
  "term_id": "GO:0005768",
  "term_label": "endosome",
  "gene": "UniProtKB:Q9Y5W9",
  "gene_name": "Sorting nexin-11"
}